{
  "gene_name": "Ras-related protein Rab-22A",
  "gene": "UniProtKB:Q9UL26",
  "gene_symbol": "RAB22A",
  "term_label": "endomembrane system",
  "term_id": "GO:0012505"
}